{
  "term_id": "GO:0051453",
  "gene_symbol": "SLC4A10",
  "gene_name": "Sodium-driven chloride bicarbonate exchanger",
  "term_label": "regulation of intracellular pH",
  "gene": "UniProtKB:Q6U841"
}